CoB-CoM heterodisulfide reductase complex [GO:0044678] (cellular component) Relationships: is a type of GO:1990204 Also known as: coenzyme M-7-mercaptoheptanoylthreonine-phosphate-heterodisulfide hydrogenase complex, hydrogen:coenzyme-M-7-mercaptoheptanoylthreonine-phosphate-heterodisulfide oxidoreductase complex Definition: A protein complex that in Methanobacterium thermoautotrophicum is composed of six subunits, and in Methanosarcina barkeri contains is composed of either two subunits or nine subunits. Catalyzes the conversion of coenzyme B, coenzyme M, and methanophenazine to form N-{7-[(2-sulfoethyl)dithio]heptanoyl}-3-O-phospho-L-threonine and dihydromethanophenazine. References: PMID:8119281, PMID:8174566, PMID:9063468 Sources: GOC:mengo_curators